{
  "gene": "UniProtKB:Q9UGI0",
  "term_id": "GO:0004843",
  "gene_name": "Ubiquitin thioesterase ZRANB1",
  "term_label": "cysteine-type deubiquitinase activity",
  "gene_symbol": "ZRANB1"
}